{
  "term_id": "GO:0017128",
  "gene_name": "Anoctamin-9",
  "term_label": "phospholipid scramblase activity",
  "gene": "UniProtKB:A1A5B4",
  "gene_symbol": "ANO9"
}